{
  "term_id": "GO:0008391",
  "term_label": "arachidonate monooxygenase activity",
  "gene_symbol": "CYP4A22",
  "gene_name": "Cytochrome P450 4A22",
  "gene": "UniProtKB:Q5TCH4"
}